lumenal side of lysosomal membrane [GO:0098575] (cellular component) Also known as: internal leaflet of lysosomal membrane, internal side of lysosomal membrane Sources: GOC:dos Relationships: is a type of lumenal side of membrane [GO:0098576]; is part of lysosomal membrane [GO:0005765] Definition: The side (leaflet) of the lysosomal membrane that faces the lumen.